{
  "gene_symbol": "SEPTIN6",
  "gene": "UniProtKB:Q14141",
  "gene_name": "Septin-6",
  "term_id": "GO:0005940",
  "term_label": "septin ring"
}